{
  "gene": "UniProtKB:Q9UF33",
  "term_id": "GO:0030425",
  "term_label": "dendrite",
  "gene_name": "Ephrin type-A receptor 6",
  "gene_symbol": "EPHA6"
}